regulation of adaptive immune memory response [GO:1905674] (biological process) Definition: Any process that modulates the frequency, rate or extent of adaptive immune memory response. References: PMID:26831526 Sources: GOC:TermGenie, GO_REF:0000058 Relationships: is a type of GO:0002819; regulates GO:0090716 Subtypes: GO:1905675, positive regulation of adaptive immune memory response [GO:1905676]